{
  "gene_name": "Protocadherin beta-7",
  "term_label": "plasma membrane",
  "term_id": "GO:0005886",
  "gene_symbol": "PCDHB7",
  "gene": "UniProtKB:Q9Y5E2"
}